{
  "term_label": "Unknown molecular function",
  "term_id": "UNKNOWN:0001",
  "gene_name": "Glutamate-rich protein 2",
  "gene": "UniProtKB:A1L162",
  "gene_symbol": "ERICH2"
}